{
  "term_label": "plasma membrane",
  "term_id": "GO:0005886",
  "gene_name": "Melanocortin-2 receptor accessory protein",
  "gene_symbol": "MRAP",
  "gene": "UniProtKB:Q8TCY5"
}